{
  "gene_symbol": "PAM",
  "term_id": "GO:0005576",
  "gene_name": "Peptidyl-glycine alpha-amidating monooxygenase",
  "gene": "UniProtKB:P19021",
  "term_label": "extracellular region"
}